{
  "term_id": "GO:0043005",
  "term_label": "neuron projection",
  "gene_symbol": "CHRNA4",
  "gene_name": "Neuronal acetylcholine receptor subunit alpha-4",
  "gene": "UniProtKB:P43681"
}